{
  "term_id": "GO:0005634",
  "term_label": "nucleus",
  "gene_symbol": "PTPN18",
  "gene_name": "Tyrosine-protein phosphatase non-receptor type 18",
  "gene": "UniProtKB:Q99952"
}